{
  "gene": "UniProtKB:P35453",
  "term_id": "GO:0006357",
  "gene_name": "Homeobox protein Hox-D13",
  "gene_symbol": "HOXD13",
  "term_label": "regulation of transcription by RNA polymerase II"
}